{
  "gene_name": "Arylsulfatase K",
  "term_id": "GO:0015024",
  "gene_symbol": "ARSK",
  "gene": "UniProtKB:Q6UWY0",
  "term_label": "glucuronate-2-sulfatase activity"
}